{
  "gene_symbol": "NFIX",
  "term_label": "regulation of transcription by RNA polymerase II",
  "gene": "UniProtKB:Q14938",
  "term_id": "GO:0006357",
  "gene_name": "Nuclear factor 1 X-type"
}